{
  "gene_name": "Histone-lysine N-methyltransferase SETD2",
  "gene": "UniProtKB:Q9BYW2",
  "term_label": "chromosome",
  "term_id": "GO:0005694",
  "gene_symbol": "SETD2"
}